symbiont-mediated suppression of host RNAi-mediated antiviral immune response [GO:0140533] (biological process) Relationships: is a type of GO:0052170 References: PMID:17693253 Definition: A process by which a symbiont inhibits or disrupts the host's RNAi-mediated antiviral immune response. The host is defined as the larger of the organisms involved in a symbiotic interaction. Also known as: suppression of host RNAi-mediated antiviral immune response, suppression of host RNAi-mediated antiviral immunity, suppression of host RNAi-mediated gene silencing